pyrimidine nucleobase biosynthetic process [GO:0019856] (BP) Definition: The chemical reactions and pathways resulting in the formation of pyrimidine nucleobases, 1,3-diazine, organic nitrogenous bases. Sources: GOC:go_curators Also known as: pyrimidine base anabolism, pyrimidine base biosynthesis, pyrimidine base biosynthetic process, pyrimidine base formation, pyrimidine base synthesis Relationships: is a type of pyrimidine nucleobase metabolic process [GO:0006206]; is a type of nucleobase biosynthetic process [GO:0046112]; is a type of GO:0072528 Subtypes: GO:0006207, pyrimidine nucleobase salvage [GO:0043100], GO:0046106, uracil biosynthetic process [GO:0046107]